{
  "term_label": "alpha-methylacyl-CoA racemase activity",
  "gene_symbol": "AMACR",
  "gene_name": "Alpha-methylacyl-CoA racemase",
  "gene": "UniProtKB:Q9UHK6",
  "term_id": "GO:0008111"
}